{
  "term_label": "Unknown biological process",
  "gene_symbol": "RNF20",
  "gene_name": "E3 ubiquitin-protein ligase BRE1A",
  "term_id": "UNKNOWN:0002",
  "gene": "UniProtKB:Q5VTR2"
}